{
  "gene_name": "ALS2 C-terminal-like protein",
  "gene": "UniProtKB:Q60I27",
  "term_label": "cytoplasm",
  "gene_symbol": "ALS2CL",
  "term_id": "GO:0005737"
}